{
  "gene_symbol": "TOR1B",
  "gene_name": "Torsin-1B",
  "term_label": "kinesin binding",
  "term_id": "GO:0019894",
  "gene": "UniProtKB:O14657"
}